outer endospore membrane [GO:0043594] (cellular component) Definition: The outer membrane around a bacterial endospore, located between the endospore cortex and endospore coat. Sources: GOC:mlg Relationships: is a type of outer membrane [GO:0019867]; is part of endospore external encapsulating structure [GO:0043591]